{
  "gene_name": "E3 ubiquitin-protein ligase RNF128",
  "gene_symbol": "RNF128",
  "term_label": "ubiquitin protein ligase activity",
  "gene": "UniProtKB:Q8TEB7",
  "term_id": "GO:0061630"
}